{
  "term_id": "GO:0007399",
  "gene": "UniProtKB:Q92796",
  "gene_symbol": "DLG3",
  "term_label": "nervous system development",
  "gene_name": "Disks large homolog 3"
}